{
  "gene": "UniProtKB:Q9Y2Q3",
  "term_label": "glutathione peroxidase activity",
  "gene_name": "Glutathione S-transferase kappa 1",
  "gene_symbol": "GSTK1",
  "term_id": "GO:0004602"
}